positive regulation of imaginal disc-derived wing size [GO:0120198] (biological process) Definition: Any process that increases the size of an imaginal disc-derived wing. Relationships: is a type of regulation of imaginal disc-derived wing size [GO:0044719] Sources: GOC:ha, PIMD:23485686